{
  "gene_symbol": "TRBC1",
  "term_label": "Unknown molecular function",
  "gene": "UniProtKB:P01850",
  "gene_name": "T cell receptor beta constant 1",
  "term_id": "UNKNOWN:0001"
}